{
  "term_id": "GO:0043138",
  "gene_symbol": "FBH1",
  "gene": "UniProtKB:Q8NFZ0",
  "term_label": "3'-5' DNA helicase activity",
  "gene_name": "F-box DNA helicase 1"
}